corazonin receptor binding [GO:0071858] (molecular function) Sources: GOC:kmv, GOC:mah Definition: Binding to a corazonin receptor. Relationships: is a type of GO:0071855